{
  "term_id": "GO:0010457",
  "gene_symbol": "CEP44",
  "gene_name": "Centrosomal protein of 44 kDa",
  "gene": "UniProtKB:Q9C0F1",
  "term_label": "centriole-centriole cohesion"
}